{
  "gene": "UniProtKB:P0C7U0",
  "gene_symbol": "ELFN1",
  "term_label": "signaling receptor activity",
  "term_id": "GO:0038023",
  "gene_name": "Protein ELFN1"
}